response to bacteriocin [GO:0046678] (biological process) Also known as: bacteriocin susceptibility/resistance Definition: Any process that results in a change in state or activity of a cell or an organism (in terms of movement, secretion, enzyme production, gene expression, etc.) as a result of a bacteriocin stimulus. A bacteriocin is a protein substance released by certain bacteria that kills but does not lyse closely related strains of bacteria. Specific bacteriocins attach to specific receptors on cell walls and induce specific metabolic block, e.g. cessation of nucleic acid or protein synthesis of oxidative phosphorylation. Sources: ISBN:0721662544 Relationships: is a type of response to antibiotic [GO:0046677]; is a type of response to nitrogen compound [GO:1901698]; is a type of response to oxygen-containing compound [GO:1901700] Subtypes: GO:0071237